{
  "gene_symbol": "RAB38",
  "term_id": "GO:0042470",
  "gene": "UniProtKB:P57729",
  "term_label": "melanosome",
  "gene_name": "Ras-related protein Rab-38"
}